glutamate synthase (NADH) activity [GO:0016040] (MF) Note: Note that this term has a MetaCyc pathway reference as the pathway only has a single step. Also known as: GOGAT activity, L-glutamate synthase activity, L-glutamate synthetase activity, L-glutamate synthase (NADH), L-glutamate:NAD+ oxidoreductase (transaminating), NADH-dependent glutamate synthase activity, NADH-glutamate synthase activity, NADH: GOGAT, glutamate (reduced nicotinamide adenine dinucleotide) synthase Definition: Catalysis of the reaction: 2 L-glutamate + NAD+ = 2-oxoglutarate + L-glutamine + H+ + NADH. Sources: EC:1.4.1.14, RHEA:13753 Relationships: is_a glutamate synthase activity [GO:0015930]